{
  "gene": "UniProtKB:Q14CN2",
  "gene_name": "Calcium-activated chloride channel regulator 4",
  "gene_symbol": "CLCA4",
  "term_id": "GO:0005229",
  "term_label": "intracellularly calcium-gated chloride channel activity"
}